{
  "gene": "UniProtKB:O15534",
  "term_id": "GO:0005737",
  "gene_symbol": "PER1",
  "gene_name": "Period circadian protein homolog 1",
  "term_label": "cytoplasm"
}